{
  "term_label": "endoplasmic reticulum",
  "term_id": "GO:0005783",
  "gene": "UniProtKB:Q96GR4",
  "gene_symbol": "ZDHHC12",
  "gene_name": "Palmitoyltransferase ZDHHC12"
}